{
  "gene_name": "Fanconi anemia core complex-associated protein 24",
  "gene": "UniProtKB:Q9BTP7",
  "term_id": "UNKNOWN:0002",
  "gene_symbol": "FAAP24",
  "term_label": "Unknown biological process"
}